{
  "term_label": "Unknown cellular component",
  "gene": "UniProtKB:Q9UKS7",
  "term_id": "UNKNOWN:0003",
  "gene_name": "Zinc finger protein Helios",
  "gene_symbol": "IKZF2"
}